calcitonin receptor activity [GO:0004948] (MF) Definition: Combining with calcitonin and transmitting the signal across the membrane by activating an associated G-protein; promotes the exchange of GDP for GTP on the alpha subunit of a heterotrimeric G-protein complex. References: PMID:21649645 Sources: GOC:mah, GOC:signaling Relationships: is a type of calcitonin family receptor activity [GO:0097642]; BFO_0000051 calcitonin binding [GO:0032841]